{
  "term_label": "extracellular space",
  "gene": "UniProtKB:P02787",
  "gene_name": "Serotransferrin",
  "gene_symbol": "TF",
  "term_id": "GO:0005615"
}